{
  "gene_symbol": "FAM83G",
  "gene_name": "Protein FAM83G",
  "gene": "UniProtKB:A6ND36",
  "term_label": "cytosol",
  "term_id": "GO:0005829"
}